{
  "gene_symbol": "KCNA10",
  "gene": "UniProtKB:Q16322",
  "gene_name": "Potassium voltage-gated channel subfamily A member 10",
  "term_label": "voltage-gated potassium channel complex",
  "term_id": "GO:0008076"
}